negative regulation of lung ciliated cell differentiation [GO:1901247] (biological process) Also known as: down regulation of lung ciliated cell differentiation, down-regulation of lung ciliated cell differentiation, downregulation of lung ciliated cell differentiation, inhibition of lung ciliated cell differentiation Relationships: is_a negative regulation of epithelial cell differentiation [GO:0030857]; is a type of negative regulation of multicellular organismal process [GO:0051241]; is a type of GO:1901246; negatively regulates lung ciliated cell differentiation [GO:0061141] Definition: Any process that stops, prevents or reduces the frequency, rate or extent of lung ciliated cell differentiation. Sources: GOC:BHF, GOC:TermGenie